UDP reductase activity [GO:0051062] (MF) Definition: Catalysis of the reaction: dUDP + thioredoxin disulfide + H2O = UDP + thioredoxin. Sources: MetaCyc:UDPREDUCT-RXN Also known as: UDP reduction Relationships: is a type of ribonucleoside-diphosphate reductase activity, thioredoxin disulfide as acceptor [GO:0004748]